{
  "gene_symbol": "CADPS",
  "term_label": "exocytosis",
  "term_id": "GO:0006887",
  "gene_name": "Calcium-dependent secretion activator 1",
  "gene": "UniProtKB:Q9ULU8"
}